{
  "gene_symbol": "SEMA3D",
  "term_id": "GO:0050919",
  "gene_name": "Semaphorin-3D",
  "term_label": "negative chemotaxis",
  "gene": "UniProtKB:O95025"
}